{
  "gene": "UniProtKB:Q03924",
  "term_id": "UNKNOWN:0003",
  "gene_name": "Zinc finger protein 117",
  "term_label": "Unknown cellular component",
  "gene_symbol": "ZNF117"
}